lysine 2-monooxygenase activity [GO:0050067] (MF) Definition: Catalysis of the reaction: L-lysine + O2 = 5-aminopentanamide + CO2 + H2O. Relationships: is a type of oxidoreductase activity, acting on single donors with incorporation of molecular oxygen, incorporation of one atom of oxygen (internal monooxygenases or internal mixed function oxidases) [GO:0016703] Sources: EC:1.13.12.2, RHEA:14601 Also known as: L-lysine-2-monooxygenase activity, L-lysine:oxygen 2-oxidoreductase (decarboxylating), lysine monooxygenase activity, lysine oxygenase activity